{
  "term_label": "cytoplasm",
  "gene": "UniProtKB:O00750",
  "gene_name": "Phosphatidylinositol 4-phosphate 3-kinase C2 domain-containing subunit beta",
  "term_id": "GO:0005737",
  "gene_symbol": "PIK3C2B"
}